{
  "gene_symbol": "MAP6",
  "gene_name": "Microtubule-associated protein 6",
  "gene": "UniProtKB:Q96JE9",
  "term_label": "dendrite",
  "term_id": "GO:0030425"
}